interleukin-7-mediated signaling pathway [GO:0038111] (biological process) Also known as: IL-7-mediated signaling pathway, interleukin-7-mediated signalling pathway Sources: GOC:nhn, GOC:signaling Definition: The series of molecular signals initiated by interleukin-7 binding to its receptor on the surface of a cell, and ending with the regulation of a downstream cellular process, e.g. transcription. Relationships: is a type of cytokine-mediated signaling pathway [GO:0019221]; is part of cellular response to interleukin-7 [GO:0098761]